{
  "gene": "UniProtKB:Q96IX9",
  "term_label": "Unknown cellular component",
  "gene_name": "Putative ankyrin repeat domain-containing protein 26-like 1",
  "gene_symbol": "ANKRD36BP1",
  "term_id": "UNKNOWN:0003"
}